{
  "gene": "UniProtKB:Q96G01",
  "gene_symbol": "BICD1",
  "term_label": "microtubule anchoring at microtubule organizing center",
  "term_id": "GO:0072393",
  "gene_name": "Protein bicaudal D homolog 1"
}